{
  "term_label": "nucleosomal DNA binding",
  "gene_symbol": "H1-0",
  "term_id": "GO:0031492",
  "gene": "UniProtKB:P07305",
  "gene_name": "Histone H1.0"
}